{
  "gene_symbol": "NTAQ1",
  "gene_name": "Protein N-terminal glutamine amidohydrolase",
  "term_id": "GO:0070773",
  "term_label": "protein-N-terminal glutamine amidohydrolase activity",
  "gene": "UniProtKB:Q96HA8"
}